regulation of renal system process [GO:0098801] (biological process) Definition: Any process that modulates the frequency, rate or extent of a system process, a multicellular organismal process carried out by the renal system. Sources: GOC:dos Relationships: is a type of regulation of system process [GO:0044057]; RO_0002211 GO:0003014 Subtypes: regulation of glomerular filtration [GO:0003093], GO:0035813, GO:1900133, regulation of renal amino acid absorption [GO:1902752], regulation of renal phosphate excretion [GO:1903402], regulation of smooth muscle contraction involved in micturition [GO:1904318], regulation of renal albumin absorption [GO:2000532], regulation of renal water transport [GO:2001151]